negative regulation of ergosterol biosynthetic process [GO:0010895] (biological process) Definition: Any process that decreases the frequency, rate or extent of the chemical reactions and pathways resulting in the formation of ergosterol. Relationships: is a type of regulation of ergosterol biosynthetic process [GO:0032443]; is a type of negative regulation of sterol biosynthetic process [GO:0106119]; is_a negative regulation of alcohol biosynthetic process [GO:1902931]; negatively regulates ergosterol biosynthetic process [GO:0006696] Sources: GOC:tb